{
  "gene_name": "Guanine nucleotide-binding protein subunit alpha-13",
  "gene_symbol": "GNA13",
  "term_label": "heterotrimeric G-protein complex",
  "gene": "UniProtKB:Q14344",
  "term_id": "GO:0005834"
}